negative regulation of B cell differentiation [GO:0045578] (biological process) Relationships: is a type of regulation of B cell differentiation [GO:0045577]; is a type of negative regulation of lymphocyte differentiation [GO:0045620]; is a type of negative regulation of B cell activation [GO:0050869]; RO_0002212 B cell differentiation [GO:0030183] Note: Note that immunologists typically use the word 'development' to refer to cells of B or T cell lineages undergoing the process that GO describes as 'cell differentiation'. Sources: GOC:go_curators Definition: Any process that stops, prevents, or reduces the frequency, rate or extent of B cell differentiation. Subtypes: negative regulation of B-1 B cell differentiation [GO:0001925], GO:0002899, negative regulation of central B cell anergy [GO:0002915], negative regulation of plasma cell differentiation [GO:1900099] Also known as: down regulation of B cell differentiation, down-regulation of B cell differentiation, downregulation of B cell differentiation, negative regulation of B lymphocyte differentiation, negative regulation of B-cell differentiation, negative regulation of B-lymphocyte differentiation, inhibition of B cell differentiation, negative regulation of B cell development